{
  "gene_symbol": "CDK2AP2",
  "term_id": "GO:0070507",
  "gene_name": "Cyclin-dependent kinase 2-associated protein 2",
  "term_label": "regulation of microtubule cytoskeleton organization",
  "gene": "UniProtKB:O75956"
}